{
  "term_id": "GO:0000981",
  "gene": "UniProtKB:Q14209",
  "gene_name": "Transcription factor E2F2",
  "gene_symbol": "E2F2",
  "term_label": "DNA-binding transcription factor activity, RNA polymerase II-specific"
}